atrial septum intermedium development [GO:0003286] (biological process) Sources: GOC:mtg_heart Definition: The progression of the atrial septum intermedium over time, from its formation to the mature structure. Relationships: is a type of atrial septum development [GO:0003283]